{
  "gene_name": "Dihydroorotate dehydrogenase (quinone), mitochondrial",
  "term_id": "GO:0004152",
  "gene": "UniProtKB:Q02127",
  "gene_symbol": "DHODH",
  "term_label": "dihydroorotate dehydrogenase activity"
}